4-formylbenzenesulfonate dehydrogenase activity [GO:0018482] (molecular function) Relationships: is a type of GO:0016620 Definition: Catalysis of the reaction: 4-formylbenzenesulfonate + H2O + NAD+ = 4-sulfobenzoate + 2 H+ + NADH. Also known as: 4-formylbenzenesulphonate dehydrogenase activity, toluene-sulfonate aldehyde dehydrogenase activity, 4-formylbenzenesulfonate:NAD+ oxidoreductase activity Sources: EC:1.2.1.62, RHEA:18833